{
  "term_label": "Unknown cellular component",
  "gene": "UniProtKB:Q15386",
  "gene_name": "Ubiquitin-protein ligase E3C",
  "term_id": "UNKNOWN:0003",
  "gene_symbol": "UBE3C"
}